positive regulation of macrophage migration inhibitory factor signaling pathway [GO:2000448] (biological process) Sources: GOC:obol Relationships: is a type of GO:0001961; is a type of GO:2000446; positively regulates macrophage migration inhibitory factor signaling pathway [GO:0035691] Also known as: positive regulation of MIF signaling pathway, positive regulation of macrophage migration inhibitory factor signalling pathway Definition: Any process that activates or increases the frequency, rate or extent of macrophage migration inhibitory factor signaling pathway.